{
  "gene": "UniProtKB:Q8N6Y2",
  "term_id": "UNKNOWN:0002",
  "term_label": "Unknown biological process",
  "gene_name": "Leucine-rich repeat-containing protein 17",
  "gene_symbol": "LRRC17"
}